{
  "gene": "UniProtKB:Q16572",
  "gene_name": "Vesicular acetylcholine transporter",
  "gene_symbol": "SLC18A3",
  "term_id": "GO:0030121",
  "term_label": "AP-1 adaptor complex"
}